{
  "term_label": "Unknown cellular component",
  "gene_symbol": "TRAV25",
  "term_id": "UNKNOWN:0003",
  "gene": "UniProtKB:A0A0B4J276",
  "gene_name": "T cell receptor alpha variable 25"
}